{
  "gene_symbol": "C18orf32",
  "gene": "UniProtKB:Q8TCD1",
  "gene_name": "UPF0729 protein C18orf32",
  "term_id": "UNKNOWN:0002",
  "term_label": "Unknown biological process"
}